snoRNA guided rRNA pseudouridine synthesis [GO:0000454] (biological process) Sources: GOC:curators, ISBN:1555811337 Definition: The intramolecular conversion of uridine to pseudouridine in an rRNA molecule during ribosome biogenesis using a snoRNA guide that targets the position of pseudouridylation. Relationships: is a type of rRNA pseudouridine synthesis [GO:0031118]